{
  "term_label": "nucleus",
  "term_id": "GO:0005634",
  "gene_name": "Phosphatidate phosphatase LPIN2",
  "gene_symbol": "LPIN2",
  "gene": "UniProtKB:Q92539"
}